regulation of T cell mediated immunity [GO:0002709] (biological process) Relationships: is a type of regulation of lymphocyte mediated immunity [GO:0002706]; is a type of regulation of adaptive immune response based on somatic recombination of immune receptors built from immunoglobulin superfamily domains [GO:0002822]; regulates T cell mediated immunity [GO:0002456] Subtypes: GO:0001807, GO:0001914, GO:0002625, negative regulation of T cell mediated immunity [GO:0002710], positive regulation of T cell mediated immunity [GO:0002711], regulation of T cell cytokine production [GO:0002724], regulation of T cell mediated immune response to tumor cell [GO:0002840], regulation of peripheral T cell tolerance induction [GO:0002849] Definition: Any process that modulates the frequency, rate, or extent of T cell mediated immunity. Also known as: regulation of T lymphocyte mediated immunity, regulation of T-cell mediated immunity, regulation of T-lymphocyte mediated immunity Sources: GOC:add